{
  "term_id": "GO:0005737",
  "term_label": "cytoplasm",
  "gene_symbol": "TAOK3",
  "gene_name": "Serine_threonine-protein kinase TAO3",
  "gene": "UniProtKB:Q9H2K8"
}